{
  "gene": "UniProtKB:A0A0B4J2E0",
  "gene_symbol": "TRBV12-4",
  "gene_name": "T cell receptor beta variable 12-4",
  "term_label": "plasma membrane",
  "term_id": "GO:0005886"
}